{
  "gene_symbol": "TRAJ5",
  "gene_name": "T cell receptor alpha joining 5 (Fragment)",
  "term_id": "UNKNOWN:0002",
  "term_label": "Unknown biological process",
  "gene": "UniProtKB:A0A075B6V8"
}